apoplast [GO:0048046] (cellular component) Sources: GOC:jid Relationships: is a type of extracellular region [GO:0005576] Definition: The cell membranes and intracellular regions in a plant are connected through plasmodesmata, and plants may be described as having two major compartments: the living symplast and the non-living apoplast. The apoplast is external to the plasma membrane and includes cell walls, intercellular spaces and the lumen of dead structures such as xylem vessels. Water and solutes pass freely through it.